{
  "gene": "UniProtKB:Q9BWM7",
  "term_id": "GO:0022857",
  "term_label": "transmembrane transporter activity",
  "gene_name": "Sideroflexin-3",
  "gene_symbol": "SFXN3"
}